positive regulation of immunoglobulin production in mucosal tissue [GO:2000558] (BP) Definition: Any process that activates or increases the frequency, rate or extent of immunoglobulin production in mucosal tissue. Sources: GOC:obol Also known as: positive regulation of antibody production in mucosal tissue Relationships: is a type of positive regulation of immunoglobulin production [GO:0002639]; is a type of GO:0002891; is a type of regulation of immunoglobulin production in mucosal tissue [GO:2000557]; positively regulates immunoglobulin production in mucosal tissue [GO:0002426]